fat pad development [GO:0060613] (biological process) Relationships: is a type of GO:0060612 Definition: The progression of a fat pad from its initial formation to its mature structure. A fat pad is an accumulation of adipose tissue. Sources: GOC:dph